{
  "gene_symbol": "ARMH2",
  "term_label": "Unknown biological process",
  "term_id": "UNKNOWN:0002",
  "gene_name": "Armadillo-like helical domain-containing protein 2",
  "gene": "UniProtKB:H3BNL8"
}